{
  "term_label": "neuron projection",
  "term_id": "GO:0043005",
  "gene_name": "N-acyl-phosphatidylethanolamine-hydrolyzing phospholipase D",
  "gene": "UniProtKB:Q6IQ20",
  "gene_symbol": "NAPEPLD"
}